tachykinin receptor signaling pathway [GO:0007217] (biological process) Relationships: is a type of G protein-coupled receptor signaling pathway [GO:0007186] Also known as: tachykinin signalling pathway Subtypes: phospholipase C-activating tachykinin receptor signaling pathway [GO:0007209] Definition: A G protein-coupled receptor signaling pathway initiated by tachykinin binding to its receptor on the surface of a target cell, and ending with the regulation of a downstream cellular process. Tachykinin is a short peptide with the terminal sequence (Phe-X-Gly-Leu-Met-NH2). References: PMID:14723970 Sources: GOC:mah